{
  "term_id": "GO:0045892",
  "term_label": "negative regulation of DNA-templated transcription",
  "gene": "UniProtKB:Q96JM7",
  "gene_symbol": "L3MBTL3",
  "gene_name": "Lethal(3)malignant brain tumor-like protein 3"
}